{
  "gene": "UniProtKB:Q5TEC6",
  "gene_name": "Histone H3-7",
  "term_id": "GO:0051382",
  "term_label": "kinetochore assembly",
  "gene_symbol": "H3-7"
}